protein methylthiotransferase activity [GO:0103039] (MF) Relationships: is a type of methylthiotransferase activity [GO:0035596]; is a type of catalytic activity, acting on a protein [GO:0140096] Definition: Catalysis of the reaction: 2 S-adenosyl-L-methionine + a [ribosomal protein S12] L-aspartate89 + a sulfurated [sulfur carrier] + a reduced electron acceptor = S-adenosyl-L-homocysteine + L-methionine + 5'-deoxyadenosine + 2 H+ + a [ribosomal protein S12] 3-methylthio-L-aspartate89 + an unsulfurated [sulfur carrier] + an oxidized electron acceptor. Sources: EC:2.8.4.4, GOC:pz